{
  "gene_name": "5'-AMP-activated protein kinase catalytic subunit alpha-2",
  "term_id": "GO:0042149",
  "gene_symbol": "PRKAA2",
  "gene": "UniProtKB:P54646",
  "term_label": "cellular response to glucose starvation"
}